GTPase complex [GO:1905360] (cellular component) Relationships: is a type of GO:1902494 Subtypes: heterotrimeric G-protein complex [GO:0005834], APC-tubulin-IQGAP1 complex [GO:0034741], APC-IQGAP complex [GO:0034743], APC-IQGAP1-Cdc42 complex [GO:0034744], APC-IQGAP1-Rac1 complex [GO:0034745], APC-IQGAP1-CLIP-170 complex [GO:0034746], Cdc42 GTPase complex [GO:0071521], Gtr1-Gtr2 GTPase complex [GO:1990131] Note: An example of this is HRAS in human (P01112) in PMID:9178006 (inferred from direct assay). References: PMID:9178006 Sources: GOC:TermGenie, GOC:bhm, GO_REF:0000088 Definition: A protein complex which is capable of GTPase activity. Also known as: HRAS-SOS1 complex, RASH-SOS1 complex